positive regulation of trichoblast fate specification [GO:0010063] (biological process) Relationships: is_a regulation of trichoblast fate specification [GO:0010061]; is a type of positive regulation of cell fate specification [GO:0042660]; is_a positive regulation of plant epidermal cell differentiation [GO:1903890]; positively regulates trichoblast fate specification [GO:0010057] Sources: GOC:tb Definition: Any process that induces or promotes trichoblast fate specification. Also known as: up regulation of trichoblast fate, up-regulation of trichoblast fate, upregulation of trichoblast fate, activation of trichoblast fate, stimulation of trichoblast fate